{
  "gene_name": "C-C motif chemokine 24",
  "term_id": "GO:0005615",
  "gene": "UniProtKB:O00175",
  "term_label": "extracellular space",
  "gene_symbol": "CCL24"
}